{
  "gene_symbol": "HSP90AB4P",
  "gene_name": "Putative heat shock protein HSP 90-beta 4",
  "gene": "UniProtKB:Q58FF6",
  "term_label": "protein folding",
  "term_id": "GO:0006457"
}